proximal/distal pattern formation involved in pronephric nephron development [GO:0072196] (biological process) Subtypes: specification of pronephric proximal tubule identity [GO:0039004], specification of pronephric distal tubule identity [GO:0039010] Sources: GOC:mtg_kidney_jan10 Definition: The regionalization process in which specific areas of cell differentiation are determined along a proximal/distal axis of the pronephros. Also known as: pronephros proximal/distal pattern formation Relationships: is a type of GO:0039017; is a type of proximal/distal pattern formation involved in nephron development [GO:0072047]; is part of pronephric nephron development [GO:0039019]